{
  "term_label": "DNA-binding transcription factor activity, RNA polymerase II-specific",
  "gene": "UniProtKB:Q969G2",
  "term_id": "GO:0000981",
  "gene_name": "LIM_homeobox protein Lhx4",
  "gene_symbol": "LHX4"
}